{
  "term_id": "GO:0015629",
  "gene_symbol": "MYO1B",
  "gene": "UniProtKB:O43795",
  "term_label": "actin cytoskeleton",
  "gene_name": "Unconventional myosin-Ib"
}